{
  "gene_name": "T-cell immunoreceptor with Ig and ITIM domains",
  "term_label": "negative regulation of interleukin-12 production",
  "term_id": "GO:0032695",
  "gene_symbol": "TIGIT",
  "gene": "UniProtKB:Q495A1"
}